{
  "gene_symbol": "SEC61A2",
  "gene_name": "Protein transport protein Sec61 subunit alpha isoform 2",
  "gene": "UniProtKB:Q9H9S3",
  "term_label": "signal sequence binding",
  "term_id": "GO:0005048"
}